MAP kinase kinase kinase kinase activity [GO:0008349] (molecular function) Definition: Catalysis of the phosphorylation of serine and threonine residues in a mitogen-activated protein kinase kinase kinase (MAPKKK), resulting in activation of MAPKKK. MAPKKK signaling pathways relay, amplify and integrate signals from the plasma membrane to the nucleus in response to a diverse range of extracellular stimuli. References: PMID:11790549 Sources: GOC:bf Also known as: MAP4K activity, MAPKKKK Relationships: is_a protein serine/threonine kinase activity [GO:0004674]; is part of MAPK cascade [GO:0000165] Subtypes: JUN kinase kinase kinase kinase activity [GO:0042656]